{
  "term_id": "GO:0005125",
  "gene_name": "Protein Wnt-10a",
  "gene": "UniProtKB:Q9GZT5",
  "gene_symbol": "WNT10A",
  "term_label": "cytokine activity"
}